establishment of protein localization to chloroplast [GO:0072596] (biological process) Subtypes: GO:0045036, protein import into chloroplast stroma [GO:0045037], protein import into chloroplast thylakoid membrane [GO:0045038] Sources: GOC:mah Relationships: is_a GO:0072594 Also known as: establishment of protein localisation to chloroplast Definition: The directed movement of a protein to a specific location in a chloroplast.